phospholactate guanylyltransferase activity [GO:0043814] (molecular function) Relationships: is a type of guanylyltransferase activity [GO:0070568] References: PMID:18260642 Sources: RHEA:63424 Definition: Catalysis of the reaction: 2-phospho-(S)-lactate + GTP = lactyl-2-diphospho-5'-guanosine + diphosphate.